{
  "gene": "UniProtKB:Q14451",
  "term_id": "GO:0035556",
  "gene_symbol": "GRB7",
  "term_label": "intracellular signal transduction",
  "gene_name": "Growth factor receptor-bound protein 7"
}